{
  "gene": "UniProtKB:Q9NZV1",
  "gene_symbol": "CRIM1",
  "gene_name": "Cysteine-rich motor neuron 1 protein",
  "term_id": "UNKNOWN:0002",
  "term_label": "Unknown biological process"
}